{
  "gene_symbol": "S100A14",
  "term_id": "GO:0071624",
  "gene": "UniProtKB:Q9HCY8",
  "term_label": "positive regulation of granulocyte chemotaxis",
  "gene_name": "Protein S100-A14"
}